{
  "term_label": "nucleus",
  "gene_name": "Zinc finger protein 34",
  "gene_symbol": "ZNF34",
  "gene": "UniProtKB:Q8IZ26",
  "term_id": "GO:0005634"
}